{
  "term_label": "late endosome membrane",
  "gene": "UniProtKB:P13473",
  "term_id": "GO:0031902",
  "gene_symbol": "LAMP2",
  "gene_name": "Lysosome-associated membrane glycoprotein 2"
}